{
  "gene_symbol": "MAST3",
  "gene_name": "Microtubule-associated serine_threonine-protein kinase 3",
  "term_id": "GO:0035556",
  "term_label": "intracellular signal transduction",
  "gene": "UniProtKB:O60307"
}